{
  "gene_symbol": "HLA-DRB3",
  "term_label": "MHC class II protein complex",
  "term_id": "GO:0042613",
  "gene_name": "HLA class II histocompatibility antigen, DR beta 3 chain",
  "gene": "UniProtKB:P79483"
}